{
  "term_id": "GO:0043523",
  "gene_symbol": "EGLN2",
  "gene_name": "Prolyl hydroxylase EGLN2",
  "gene": "UniProtKB:Q96KS0",
  "term_label": "regulation of neuron apoptotic process"
}